negative regulation of membrane potential [GO:0045837] (biological process) Also known as: down regulation of membrane potential, down-regulation of membrane potential, downregulation of membrane potential, reduction of membrane potential, inhibition of membrane potential Relationships: is a type of regulation of membrane potential [GO:0042391] Sources: GOC:go_curators Subtypes: negative regulation of mitochondrial membrane potential [GO:0010917] Definition: Any process that stops, prevents, or reduces the frequency, rate or extent of establishment or extent of a membrane potential, the electric potential existing across any membrane arising from charges in the membrane itself and from the charges present in the media on either side of the membrane.